protein-N-terminal glutamine amidohydrolase activity [GO:0070773] (molecular function) Relationships: is_a GO:0016811; is a type of catalytic activity, acting on a protein [GO:0140096] Also known as: NtQ-amidase activity Definition: Catalysis of the reaction: N-terminal L-glutaminyl-[protein] + H2O = N-terminal L-glutamyl-[protein] + NH3. This reaction is the deamidation of an N-terminal glutamine residue of a protein. References: PMID:19560421 Sources: RHEA:50680